{
  "term_id": "GO:0015275",
  "gene": "UniProtKB:O75949",
  "term_label": "stretch-activated, monoatomic cation-selective, calcium channel activity",
  "gene_name": "NALCN channel auxiliary factor 2",
  "gene_symbol": "NALF2"
}